negative regulation of brassinosteroid mediated signaling pathway [GO:1900458] (BP) Relationships: is_a negative regulation of signal transduction [GO:0009968]; is a type of regulation of brassinosteroid mediated signaling pathway [GO:1900457]; negatively regulates brassinosteroid mediated signaling pathway [GO:0009742] Definition: Any process that stops, prevents or reduces the frequency, rate or extent of brassinosteroid mediated signaling pathway. Also known as: down regulation of brassinosteroid mediated signaling pathway, down regulation of brassinosteroid mediated signalling, down-regulation of brassinosteroid mediated signaling pathway, down-regulation of brassinosteroid mediated signalling, downregulation of brassinosteroid mediated signaling pathway, downregulation of brassinosteroid mediated signalling, inhibition of brassinosteroid mediated signalling, negative regulation of brassinosteroid mediated signalling, inhibition of brassinosteroid mediated signaling pathway References: PMID:21855796 Sources: GOC:TermGenie